{
  "term_label": "GTPase activity",
  "gene_symbol": "GBP1",
  "term_id": "GO:0003924",
  "gene_name": "Guanylate-binding protein 1",
  "gene": "UniProtKB:P32455"
}